phenol-containing compound metabolic process [GO:0018958] (biological process) Sources: ISBN:0198506732 Definition: The chemical reactions and pathways involving a phenol, any compound containing one or more hydroxyl groups directly attached to an aromatic carbon ring. Note: Note that phenol metabolism is not included as a child of 'xenobiotic metabolism' because although it is synthesized industrially, phenol is also found naturally in animal wastes and other organic materials. It is often formed by the activity of microorganisms, which can chemically modify a variety of xenobiotic and naturally occurring phenolic compounds. Relationships: is a type of metabolic process [GO:0008152] Subtypes: melanin metabolic process [GO:0006582], salicylic acid metabolic process [GO:0009696], catechol-containing compound metabolic process [GO:0009712], GO:0018881, 3-hydroxybenzyl alcohol metabolic process [GO:0018921], 4-nitrophenol metabolic process [GO:0018960], GO:0018982, phenol-containing compound catabolic process [GO:0019336], resorcinol metabolic process [GO:0019505], 1-(3,5-dichloro-2,6-dihydroxy-4-methoxyphenyl)hexan-1-one metabolic process [GO:0031147], ferulate metabolic process [GO:0033494], asperthecin metabolic process [GO:0036182], anaerobic phenol-containing compound metabolic process [GO:0042215], thyroid hormone metabolic process [GO:0042403], serotonin metabolic process [GO:0042428], GO:0042854, phenol-containing compound biosynthetic process [GO:0046189], GO:0046333, GO:1900570, GO:1900813, 4-hydroxyphenylacetate metabolic process [GO:1901022], (-)-pinoresinol metabolic process [GO:1901598], GO:1901709 Also known as: carbolic acid metabolic process, carbolic acid metabolism, hydroxybenzene metabolic process, hydroxybenzene metabolism, phenol-containing compound metabolism